{
  "gene_symbol": "TGFB3",
  "gene": "UniProtKB:P10600",
  "term_label": "extracellular space",
  "gene_name": "Transforming growth factor beta-3 proprotein",
  "term_id": "GO:0005615"
}